{
  "term_label": "NatA complex",
  "term_id": "GO:0031415",
  "gene_name": "N-alpha-acetyltransferase 15, NatA auxiliary subunit",
  "gene": "UniProtKB:Q9BXJ9",
  "gene_symbol": "NAA15"
}